{
  "term_label": "synaptic transmission, glutamatergic",
  "gene": "UniProtKB:Q9ULK0",
  "gene_symbol": "GRID1",
  "term_id": "GO:0035249",
  "gene_name": "Glutamate receptor ionotropic, delta-1"
}